negative regulation of hemocyte proliferation [GO:0035207] (biological process) Relationships: is a type of GO:0002683; is a type of negative regulation of cell population proliferation [GO:0008285]; is a type of regulation of hemocyte proliferation [GO:0035206]; negatively regulates hemocyte proliferation [GO:0035172] Sources: GOC:bf, GOC:mtg_sensu Definition: Any process that stops, prevents or reduces the rate or extent of hemocyte proliferation. Hemocytes are blood cells associated with a hemocoel (the cavity containing most of the major organs of the arthropod body) which are involved in defense and clotting of hemolymph, but not involved in transport of oxygen. An example of this is found in Drosophila melanogaster. Also known as: down regulation of hemocyte proliferation, down-regulation of hemocyte proliferation, downregulation of hemocyte proliferation, negative regulation of arthropod blood cell proliferation, inhibition of hemocyte proliferation